all-trans-undecaprenyl-phosphate mannosyltransferase activity [GO:0036427] (MF) Sources: RHEA:28118 Definition: Catalysis of the reaction: all-trans-undecaprenyl phosphate + GDP-alpha-D-mannose = D-mannosyl undecaprenyl phosphate + GDP. Relationships: is a type of GO:0047267